{
  "term_id": "UNKNOWN:0001",
  "term_label": "Unknown molecular function",
  "gene_symbol": "VWA5A",
  "gene_name": "von Willebrand factor A domain-containing protein 5A",
  "gene": "UniProtKB:O00534"
}